cell-cell self recognition [GO:0097656] (BP) Note: Examples are the membrane proteins TgrB1 and TgrC1 in the social amoeba Dictyostelium discoideum. References: PMID:21700835, PMID:23910661 Sources: GOC:pf Definition: A cell-cell recognition process by which a cell distinguishes between self and non self during cooperative behavior, such as early development. Relationships: is a type of cell-cell recognition [GO:0009988] Also known as: kin recognition, self recognition, kin discrimination